{
  "term_id": "GO:0050911",
  "gene_name": "Olfactory receptor 2A7",
  "term_label": "detection of chemical stimulus involved in sensory perception of smell",
  "gene": "UniProtKB:Q96R45",
  "gene_symbol": "OR2A7"
}